{
  "gene": "UniProtKB:Q14934",
  "term_label": "positive regulation of transcription by RNA polymerase II",
  "gene_symbol": "NFATC4",
  "term_id": "GO:0045944",
  "gene_name": "Nuclear factor of activated T-cells, cytoplasmic 4"
}